negative regulation of infection cushion formation [GO:0075186] (biological process) Sources: GOC:pamgo_curators Also known as: negative regulation of infection cushion formation on or near host Definition: Any process that stops, prevents, or reduces the frequency, rate or extent of symbiont infection cushion formation on or near its host organism. The host is defined as the larger of the organisms involved in a symbiotic interaction. Relationships: is_a negative regulation of developmental process [GO:0051093]; is a type of regulation of infection cushion formation [GO:0075184]; negatively regulates infection cushion formation [GO:0075183]